{
  "gene": "UniProtKB:Q8NCE0",
  "gene_symbol": "TSEN2",
  "term_label": "tRNA processing",
  "term_id": "GO:0008033",
  "gene_name": "tRNA-splicing endonuclease subunit Sen2"
}